neurofilament cytoskeleton organization [GO:0060052] (biological process) Definition: A process that is carried out at the cellular level which results in the assembly, arrangement of constituent parts, or disassembly of cytoskeletal structures comprising neurofilaments and their associated proteins. Relationships: is a type of intermediate filament cytoskeleton organization [GO:0045104] Sources: GOC:dph Also known as: neurofilament cytoskeleton organisation, neurofilament cytoskeleton organization and biogenesis